sulfiredoxin activity [GO:0032542] (molecular function) Definition: Catalysis of the reaction: peroxiredoxin-(S-hydroxy-S-oxocysteine) + ATP + 2 R-SH = peroxiredoxin-(S-hydroxycysteine) + ADP + phosphate + R-S-S-R. Relationships: is a type of antioxidant activity [GO:0016209]; is a type of oxidoreductase activity, acting on a sulfur group of donors [GO:0016667] References: PMID:16102934 Sources: EC:1.8.98.2 Also known as: peroxiredoxin-(S-hydroxy-S-oxocysteine) reductase activity, sulphiredoxin activity, Srx1, peroxiredoxin-(S-hydroxy-S-oxocysteine):thiol oxidoreductase [ATP-hydrolysing; peroxiredoxin-(S-hydroxycysteine)-forming]